{
  "term_id": "GO:0008013",
  "gene_symbol": "AMER2",
  "gene": "UniProtKB:Q8N7J2",
  "term_label": "beta-catenin binding",
  "gene_name": "APC membrane recruitment protein 2"
}